spermidine import across plasma membrane [GO:0140203] (biological process) Relationships: is a type of polyamine import across plasma membrane [GO:0140202]; is_a spermidine transmembrane transport [GO:1903711] Sources: GOC:vw Definition: The directed movement of spermidine from outside of a cell, across the plasma membrane and into the cytosol.